{
  "gene_symbol": "C1QBP",
  "term_id": "GO:0001849",
  "gene": "UniProtKB:Q07021",
  "gene_name": "Complement component 1 Q subcomponent-binding protein, mitochondrial",
  "term_label": "complement component C1q complex binding"
}